{
  "gene_name": "Leucine-rich repeat-containing protein 14B",
  "gene": "UniProtKB:A6NHZ5",
  "term_id": "UNKNOWN:0002",
  "gene_symbol": "LRRC14B",
  "term_label": "Unknown biological process"
}